cell-cell junction disassembly [GO:0150147] (biological process) Relationships: is a type of cell-cell junction organization [GO:0045216]; is a type of cell junction disassembly [GO:0150146] Definition: The disaggregation of a cell-cell junction into its constituent components. References: PMID:25490267 Sources: GOC:aruk Subtypes: desmosome disassembly [GO:0035921], adherens junction disassembly [GO:0120179], tight junction disassembly [GO:1905071]